{
  "gene": "UniProtKB:Q9UKN7",
  "term_id": "GO:0015629",
  "gene_symbol": "MYO15A",
  "gene_name": "Unconventional myosin-XV",
  "term_label": "actin cytoskeleton"
}